1-alkenyl-2-acylglycerol choline phosphotransferase activity [GO:0047359] (molecular function) Definition: Catalysis of the reaction: 1-alkenyl-2-acylglycerol + CDP-choline = plasmenylcholine + CMP. Relationships: is a type of GO:0016780 Sources: EC:2.7.8.22, MetaCyc:2.7.8.22-RXN Also known as: CDP-choline-1-alkenyl-2-acyl-glycerol phosphocholinetransferase activity, CDP-choline:1-alkenyl-2-acylglycerol cholinephosphotransferase activity